negative regulation of cell killing [GO:0031342] (biological process) Relationships: is a type of regulation of cell killing [GO:0031341]; is a type of negative regulation of cellular process [GO:0048523]; negatively regulates cell killing [GO:0001906] Subtypes: negative regulation of leukocyte mediated cytotoxicity [GO:0001911], negative regulation of killing of cells of another organism [GO:0051711], negative regulation of complement-dependent cytotoxicity [GO:1903660] Sources: GOC:mah Also known as: down regulation of cell killing, down-regulation of cell killing, downregulation of cell killing, inhibition of cell killing Definition: Any process that stops, prevents, or reduces the frequency, rate or extent of cell killing.